hippocampal pyramidal neuron differentiation [GO:0097432] (biological process) Relationships: is a type of GO:0021859; is a type of cerebral cortex neuron differentiation [GO:0021895] Definition: The process in which a relatively unspecialized cell acquires specialized features of a hippocampal pyramidal neuron, a pyramidal cell of the hippocampus. References: PMID:19342486 Sources: CL:1001571, GOC:jc